{
  "term_label": "innate immune response",
  "gene": "UniProtKB:P59665",
  "gene_name": "Neutrophil defensin 1",
  "gene_symbol": "DEFA1B",
  "term_id": "GO:0045087"
}